ryanodine-sensitive calcium-release channel activity involved in regulation of postsynaptic cytosolic calcium levels [GO:0098697] (molecular function) Definition: Any ryanodine-sensitive calcium-release channel activity that is involved in regulation of postsynaptic cytosolic calcium ion concentration. Sources: GOC:dos Relationships: is a type of ryanodine-sensitive calcium-release channel activity [GO:0005219]; is a type of GO:1905058